{
  "term_id": "UNKNOWN:0001",
  "gene": "UniProtKB:Q9UKT5",
  "term_label": "Unknown molecular function",
  "gene_symbol": "FBXO4",
  "gene_name": "F-box only protein 4"
}